{
  "term_label": "Unknown biological process",
  "gene_symbol": "CCNL2",
  "term_id": "UNKNOWN:0002",
  "gene_name": "Cyclin-L2",
  "gene": "UniProtKB:Q96S94"
}